{
  "term_label": "nucleus",
  "gene": "UniProtKB:Q92989",
  "term_id": "GO:0005634",
  "gene_name": "Polyribonucleotide 5'-hydroxyl-kinase Clp1",
  "gene_symbol": "CLP1"
}